negative regulation of sulfur utilization [GO:0045882] (BP) Relationships: is a type of GO:0006792; is a type of GO:0032108; negatively regulates GO:0006791 Definition: Any process that stops, prevents, or reduces the frequency, rate or extent of sulfur utilization. Also known as: down regulation of sulfur utilization, down-regulation of sulfur utilization, downregulation of sulfur utilization, negative regulation of sulphur utilization, inhibition of sulfur utilization Sources: GOC:go_curators